{
  "gene_name": "Cyclin-Q",
  "term_id": "UNKNOWN:0002",
  "gene": "UniProtKB:Q8N1B3",
  "gene_symbol": "CCNQ",
  "term_label": "Unknown biological process"
}